{
  "gene": "UniProtKB:Q9H707",
  "term_id": "GO:0000981",
  "gene_name": "Zinc finger protein 552",
  "term_label": "DNA-binding transcription factor activity, RNA polymerase II-specific",
  "gene_symbol": "ZNF552"
}